{
  "gene": "UniProtKB:Q13586",
  "term_id": "GO:0005886",
  "gene_symbol": "STIM1",
  "gene_name": "Stromal interaction molecule 1",
  "term_label": "plasma membrane"
}